regulation of oxygen metabolic process [GO:2000374] (biological process) Also known as: regulation of diatomic oxygen metabolic process, regulation of oxygen metabolism Sources: GOC:mah Definition: Any process that modulates the frequency, rate or extent of oxygen metabolic process. Relationships: is a type of regulation of metabolic process [GO:0019222]; regulates oxygen metabolic process [GO:0072592]